{
  "gene_name": "E3 ubiquitin-protein ligase UHRF2",
  "term_id": "UNKNOWN:0003",
  "gene_symbol": "UHRF2",
  "gene": "UniProtKB:Q96PU4",
  "term_label": "Unknown cellular component"
}